{
  "gene_name": "Nucleolar RNA helicase 2",
  "term_label": "nucleolus",
  "gene_symbol": "DDX21",
  "gene": "UniProtKB:Q9NR30",
  "term_id": "GO:0005730"
}